{
  "gene_symbol": "VDAC3",
  "gene": "UniProtKB:Q9Y277",
  "term_id": "UNKNOWN:0002",
  "gene_name": "Voltage-dependent anion-selective channel protein 3",
  "term_label": "Unknown biological process"
}